cellular response to lithium ion [GO:0071285] (biological process) Sources: GOC:mah Relationships: is a type of GO:0010226; is a type of GO:0071248 Definition: Any process that results in a change in state or activity of a cell (in terms of movement, secretion, enzyme production, gene expression, etc.) as a result of a lithium (Li+) ion stimulus.